{
  "gene": "UniProtKB:Q02763",
  "term_label": "endothelial cell proliferation",
  "gene_name": "Angiopoietin-1 receptor",
  "gene_symbol": "TEK",
  "term_id": "GO:0001935"
}